{
  "term_label": "chylomicron",
  "gene_symbol": "APOE",
  "gene": "UniProtKB:P02649",
  "term_id": "GO:0042627",
  "gene_name": "Apolipoprotein E"
}